{
  "gene_symbol": "MT1G",
  "term_label": "detoxification of copper ion",
  "gene": "UniProtKB:P13640",
  "term_id": "GO:0010273",
  "gene_name": "Metallothionein-1G"
}